{
  "gene_symbol": "MMP16",
  "gene_name": "Matrix metalloproteinase-16",
  "term_label": "extracellular matrix organization",
  "gene": "UniProtKB:P51512",
  "term_id": "GO:0030198"
}